proximal convoluted tubule segment 2 development [GO:0072032] (biological process) Definition: The process whose specific outcome is the progression of the S2 portion of the proximal convoluted tubule over time, from its formation to the mature structure. The S2 portion of the tubule is involved in reabsorption of water and sodium chloride. Sources: GOC:mtg_kidney_jan10, MA:0002613 Also known as: S2 development Relationships: is a type of GO:0035295; is part of proximal convoluted tubule development [GO:0072019] Subtypes: metanephric proximal convoluted tubule segment 2 development [GO:0072232]